nitrate import [GO:1902025] (BP) References: PMID:22658680 Sources: GOC:TermGenie Subtypes: GO:0015706 Relationships: is a type of inorganic anion transport [GO:0015698]; is a type of GO:0071705 Also known as: nitrate influx, nitrate uptake Definition: The directed movement of nitrate into a cell or organelle.